{
  "gene_name": "Serine_threonine-protein phosphatase 2B catalytic subunit beta isoform",
  "gene": "UniProtKB:P16298",
  "term_id": "GO:0005516",
  "term_label": "calmodulin binding",
  "gene_symbol": "PPP3CB"
}